salicylic acid mediated signaling pathway [GO:0009863] (biological process) Relationships: is a type of signal transduction [GO:0007165]; is part of cellular response to salicylic acid stimulus [GO:0071446] Sources: GOC:jy Definition: The series of molecular signals mediated by salicylic acid. Also known as: salicylic acid mediated signal transduction, salicylic acid mediated signalling pathway, salicylic acid-mediated signaling pathway Subtypes: systemic acquired resistance, salicylic acid mediated signaling pathway [GO:0009862] Regulation: positively regulated by positive regulation of salicylic acid mediated signaling pathway [GO:0080151]; regulated by GO:2000031